{
  "gene_symbol": "DNM1P46",
  "term_label": "Unknown biological process",
  "gene_name": "Putative GED domain-containing protein DNM1P46",
  "term_id": "UNKNOWN:0002",
  "gene": "UniProtKB:Q6ZS02"
}